regulation of flagellated sperm motility [GO:1901317] (biological process) Definition: Any process that modulates the frequency, rate or extent of flagellated sperm motility. Relationships: is_a regulation of cilium movement involved in cell motility [GO:0060295]; is a type of regulation of reproductive process [GO:2000241]; RO_0002211 GO:0030317 Sources: GOC:TermGenie, GOC:cilia, GOC:krc Also known as: regulation of sperm motility, regulation of sperm movement Subtypes: negative regulation of flagellated sperm motility [GO:1901318], positive regulation of flagellated sperm motility [GO:1902093]